{
  "gene_name": "Fc receptor-like protein 4",
  "term_id": "GO:0007166",
  "gene": "UniProtKB:Q96PJ5",
  "term_label": "cell surface receptor signaling pathway",
  "gene_symbol": "FCRL4"
}